{
  "term_id": "GO:0051879",
  "term_label": "Hsp90 protein binding",
  "gene": "UniProtKB:Q96M98",
  "gene_name": "Parkin coregulated gene protein",
  "gene_symbol": "PACRG"
}